{
  "term_label": "plasma membrane",
  "gene": "UniProtKB:Q6UXL0",
  "gene_name": "Interleukin-20 receptor subunit beta",
  "term_id": "GO:0005886",
  "gene_symbol": "IL20RB"
}